digestion [GO:0007586] (biological process) Subtypes: lipid digestion [GO:0044241], polysaccharide digestion [GO:0044245], protein digestion [GO:0044256] Relationships: is a type of GO:0032501 Sources: GOC:isa_complete, ISBN:0198506732 Definition: The whole of the physical, chemical, and biochemical processes carried out by multicellular organisms to break down ingested nutrients into components that may be easily absorbed and directed into metabolism.